{
  "gene": "UniProtKB:A0A075B6V5",
  "term_label": "Unknown molecular function",
  "gene_name": "T cell receptor alpha variable 36_delta variable 7",
  "term_id": "UNKNOWN:0001",
  "gene_symbol": "TRAV36DV7"
}